{
  "gene_symbol": "PRG3",
  "gene": "UniProtKB:Q9Y2Y8",
  "term_label": "Unknown molecular function",
  "gene_name": "Proteoglycan 3",
  "term_id": "UNKNOWN:0001"
}